{
  "gene": "UniProtKB:P45379",
  "term_id": "GO:0030172",
  "term_label": "troponin C binding",
  "gene_symbol": "TNNT2",
  "gene_name": "Troponin T, cardiac muscle"
}